{
  "gene_name": "Protein FAM216B",
  "term_label": "Unknown molecular function",
  "term_id": "UNKNOWN:0001",
  "gene_symbol": "FAM216B",
  "gene": "UniProtKB:Q8N7L0"
}